{
  "gene_symbol": "MAP3K3",
  "term_label": "MAPK cascade",
  "gene_name": "Mitogen-activated protein kinase kinase kinase 3",
  "gene": "UniProtKB:Q99759",
  "term_id": "GO:0000165"
}